{
  "term_id": "GO:0005615",
  "gene_name": "Regenerating islet-derived protein 3-gamma",
  "gene_symbol": "REG3G",
  "gene": "UniProtKB:Q6UW15",
  "term_label": "extracellular space"
}